{
  "term_id": "GO:0005634",
  "gene_symbol": "ZCWPW2",
  "gene_name": "Zinc finger CW-type PWWP domain protein 2",
  "term_label": "nucleus",
  "gene": "UniProtKB:Q504Y3"
}